{
  "gene_name": "Beta-1,4-galactosyltransferase 2",
  "term_label": "Unknown biological process",
  "gene": "UniProtKB:O60909",
  "term_id": "UNKNOWN:0002",
  "gene_symbol": "B4GALT2"
}